{
  "gene_symbol": "TSPY2",
  "term_label": "Unknown biological process",
  "gene_name": "Testis-specific Y-encoded protein 2",
  "gene": "UniProtKB:A6NKD2",
  "term_id": "UNKNOWN:0002"
}